{
  "gene": "UniProtKB:Q7Z3K6",
  "term_id": "GO:0042826",
  "term_label": "histone deacetylase binding",
  "gene_symbol": "MIER3",
  "gene_name": "Mesoderm induction early response protein 3"
}